{
  "gene_symbol": "BMPR2",
  "gene_name": "Bone morphogenetic protein receptor type-2",
  "term_id": "GO:0030509",
  "term_label": "BMP signaling pathway",
  "gene": "UniProtKB:Q13873"
}